genkwanin 6-hydroxylase activity [GO:0102532] (molecular function) Sources: RHEA:73427 Definition: Catalysis of the reaction: genkwanin + O2 + reduced [NADPH--hemoprotein reductase] = H2O + oxidized [NADPH--hemoprotein reductase] + scutellarein 7-methyl ether. Relationships: is a type of oxidoreductase activity, acting on paired donors, with incorporation or reduction of molecular oxygen, NAD(P)H as one donor, and incorporation of one atom of oxygen [GO:0016709]